response to pH [GO:0009268] (biological process) Relationships: is a type of response to abiotic stimulus [GO:0009628] Subtypes: response to alkaline pH [GO:0010446], response to acidic pH [GO:0010447], response to neutral pH [GO:0036176], filamentous growth of a population of unicellular organisms in response to pH [GO:0036177], cellular response to pH [GO:0071467] Sources: GOC:jl, Wikipedia:PH Definition: Any process that results in a change in state or activity of a cell or an organism (in terms of movement, secretion, enzyme production, gene expression, etc.) as a result of a pH stimulus. pH is a measure of the acidity or basicity of an aqueous solution.